endoplasmic reticulum membrane-lipid droplet contact site [GO:0160259] (cellular component) Definition: A membrane contact site between the endoplasmic reticulum (ER) membrane and the lipid droplet. References: PMID:24497546, PMID:30523332, PMID:37150040 Also known as: ER-LD contact site, bridging endoplasmic reticulum-lipid droplet contact Relationships: is a type of GO:0110165